{
  "term_label": "extracellular matrix",
  "term_id": "GO:0031012",
  "gene_name": "Metalloproteinase inhibitor 1",
  "gene": "UniProtKB:P01033",
  "gene_symbol": "TIMP1"
}